{
  "gene": "UniProtKB:O15550",
  "gene_name": "Lysine-specific demethylase 6A",
  "gene_symbol": "KDM6A",
  "term_id": "GO:0071558",
  "term_label": "histone H3K27me2/H3K27me3 demethylase activity"
}